{
  "gene": "UniProtKB:O75934",
  "gene_symbol": "BCAS2",
  "term_label": "catalytic step 2 spliceosome",
  "term_id": "GO:0071013",
  "gene_name": "Pre-mRNA-splicing factor SPF27"
}